extrinsic component of postsynaptic membrane [GO:0098890] (CC) Sources: GOC:autophagy, GOC:mf Relationships: is a type of extrinsic component of synaptic membrane [GO:0099243]; is part of GO:0045211 Definition: The component of the postsynaptic membrane consisting of gene products and protein complexes that are loosely bound to one of its surfaces, but not integrated into the hydrophobic region. Subtypes: GO:0098892, GO:0098893